chrysobactin transport [GO:0042932] (biological process) References: PMID:8837459 Sources: GOC:jl Relationships: is a type of organic hydroxy compound transport [GO:0015850]; is a type of siderophore transport [GO:0015891]; is a type of dipeptide transport [GO:0042938]; is a type of carboxylic acid transport [GO:0046942] Definition: The directed movement of the siderophore chrysobactin (alpha-N-(2,3-dihydroxybenzoyl)-D-lysyl-L-serine) into, out of or within a cell, or between cells, by means of some agent such as a transporter or pore.